4-O-methyl-glucuronoyl methylesterase activity [GO:0052797] (molecular function) Also known as: glucuronoyl esterase activity References: PMID:16876163 Sources: GOC:mengo_curators Definition: Catalysis of the reaction: [X]-4-O-methyl-D-glucuronic acid + H2O = [X]-OH + methyl-D-glucuronic acid. This reaction is the hydrolysis of the ester linkage between 4-O-methyl-D-glucuronic acid (MeGlcA) and an alcohol (-OH) group attached to a molecule, denoted here as [X]. Relationships: is a type of carboxylic ester hydrolase activity [GO:0052689]